aldose reductase (NADPH) activity [GO:0004032] (molecular function) Definition: Catalysis of the reaction: an alditol + NADP+ = an aldose + NADPH + H+. Subtypes: D-xylose reductase (NADPH) activity [GO:0032866], GO:0032867 Also known as: alditol:NADP+ 1-oxidoreductase activity, aldehyde reductase activity, aldose reductase activity, polyol dehydrogenase (NADP(+)) activity Sources: EC:1.1.1.21 Relationships: is a type of alcohol dehydrogenase (NADP+) activity [GO:0008106]